{
  "term_label": "G protein-coupled receptor signaling pathway",
  "gene_name": "Olfactory receptor 8D1",
  "term_id": "GO:0007186",
  "gene": "UniProtKB:Q8WZ84",
  "gene_symbol": "OR8D1"
}